pyramidal neuron development [GO:0021860] (biological process) Sources: GOC:cls, GOC:dgh, GOC:dph, GOC:jid, GO_REF:0000021 Definition: The progression of a pyramidal neuron from its initial formation to its mature state. Relationships: is a type of forebrain neuron development [GO:0021884]; is part of pyramidal neuron differentiation [GO:0021859] Also known as: projection neuron development